{
  "gene": "UniProtKB:P02795",
  "term_id": "GO:0071280",
  "gene_symbol": "MT2A",
  "term_label": "cellular response to copper ion",
  "gene_name": "Metallothionein-2"
}